{
  "term_label": "Unknown cellular component",
  "term_id": "UNKNOWN:0003",
  "gene_name": "Zinc finger protein 280B",
  "gene_symbol": "ZNF280B",
  "gene": "UniProtKB:Q86YH2"
}